atrial cardiac muscle cell to AV node cell signaling [GO:0086026] (biological process) Relationships: is a type of cell-cell signaling involved in cardiac conduction [GO:0086019]; is a type of GO:0086066 Definition: Any process that mediates the transfer of information from an atrial cardiomyocyte to an AV node cell. Sources: GOC:BHF, GOC:mtg_cardiac_conduct_nov11 Also known as: atrial cardiomyocyte to AV node cell signaling, atrial cardiomyocyte to AV node cell signalling, atrial cardiomyocyte to atrioventricular node cell signaling